cytochrome-b5 reductase activity, acting on NAD(P)H [GO:0004128] (molecular function) Relationships: is a type of oxidoreductase activity, acting on NAD(P)H, heme protein as acceptor [GO:0016653] Sources: GOC:curators Subtypes: cytochrome-b5 reductase activity, acting on NADPH [GO:0090523], GO:0090524 Definition: Catalysis of the reaction: 2 Fe(III)-[cytochrome b5] + NAD(P)H = 2 Fe(II)-[cytochrome b5] + NAD(P)+ + H+.